{
  "gene": "UniProtKB:O75452",
  "term_label": "retinol metabolic process",
  "gene_symbol": "RDH16",
  "term_id": "GO:0042572",
  "gene_name": "Retinol dehydrogenase 16"
}